{
  "term_label": "cell migration",
  "gene_name": "Integrin beta-4",
  "term_id": "GO:0016477",
  "gene": "UniProtKB:P16144",
  "gene_symbol": "ITGB4"
}